{
  "gene_symbol": "NRBP2",
  "term_label": "cytosol",
  "term_id": "GO:0005829",
  "gene": "UniProtKB:Q9NSY0",
  "gene_name": "Nuclear receptor-binding protein 2"
}